potassium:proton antiporter activity [GO:0015386] (molecular function) Also known as: potassium:hydrogen antiporter activity Relationships: is a type of GO:0022821; is a type of metal cation:proton antiporter activity [GO:0051139] Sources: TC:2.A.37.-.- Definition: Enables the transfer of a solute or solutes from one side of a membrane to the other according to the reaction: K+(in) + H+(out) = K+(out) + H+(in).